signal transduction involved in filamentous growth [GO:0001402] (biological process) References: PMID:9728395 Sources: GOC:mcc Definition: Relaying of environmental signals promoting filamentous growth. Also known as: MAPKKK cascade (pseudohyphal growth), signal transduction during filamentous growth Relationships: is_a signal transduction [GO:0007165]; is part of filamentous growth [GO:0030447]